{
  "gene_name": "Junctional cadherin 5-associated protein",
  "gene_symbol": "JCAD",
  "term_id": "UNKNOWN:0001",
  "gene": "UniProtKB:Q9P266",
  "term_label": "Unknown molecular function"
}